{
  "term_label": "Unknown biological process",
  "gene_symbol": "C11orf42",
  "term_id": "UNKNOWN:0002",
  "gene": "UniProtKB:Q8N5U0",
  "gene_name": "Uncharacterized protein C11orf42"
}